plastid outer membrane [GO:0009527] (cellular component) Definition: The outer, i.e. cytoplasm-facing, lipid bilayer of the plastid envelope. Sources: GOC:lr Relationships: is a type of organelle outer membrane [GO:0031968]; is a type of GO:0042170 Subtypes: GO:0009707, GO:0031900, cyanelle outer membrane [GO:0036013]